{
  "term_label": "cytosol",
  "gene_name": "Rho-related GTP-binding protein RhoN",
  "gene": "UniProtKB:P52198",
  "term_id": "GO:0005829",
  "gene_symbol": "RND2"
}